{
  "gene": "UniProtKB:Q6UXL0",
  "gene_name": "Interleukin-20 receptor subunit beta",
  "gene_symbol": "IL20RB",
  "term_id": "GO:0019221",
  "term_label": "cytokine-mediated signaling pathway"
}